{
  "gene_symbol": "LRP5",
  "gene_name": "Low-density lipoprotein receptor-related protein 5",
  "term_label": "Unknown cellular component",
  "gene": "UniProtKB:O75197",
  "term_id": "UNKNOWN:0003"
}